{
  "gene_symbol": "NPAS2",
  "term_id": "GO:0032922",
  "term_label": "circadian regulation of gene expression",
  "gene": "UniProtKB:Q99743",
  "gene_name": "Neuronal PAS domain-containing protein 2"
}